{
  "gene": "UniProtKB:Q15569",
  "term_label": "actin cytoskeleton organization",
  "term_id": "GO:0030036",
  "gene_symbol": "TESK1",
  "gene_name": "Dual specificity testis-specific protein kinase 1"
}